{
  "gene_name": "PHD finger protein 1",
  "term_label": "nucleus",
  "term_id": "GO:0005634",
  "gene_symbol": "PHF1",
  "gene": "UniProtKB:O43189"
}